{
  "gene": "UniProtKB:Q5VT06",
  "term_label": "Unknown biological process",
  "term_id": "UNKNOWN:0002",
  "gene_name": "Centrosome-associated protein 350",
  "gene_symbol": "CEP350"
}